negative regulation of excitatory postsynaptic potential [GO:0090394] (biological process) Subtypes: negative regulation of mini excitatory postsynaptic potential [GO:0061886] Definition: Any process that prevents the establishment or decreases the extent of the excitatory postsynaptic potential (EPSP) which is a temporary increase in postsynaptic potential due to the flow of positively charged ions into the postsynaptic cell. The flow of ions that causes an EPSP is an excitatory postsynaptic current (EPSC) and makes it easier for the neuron to fire an action potential. Relationships: is a type of GO:0048519; is a type of GO:0098815; negatively regulates GO:0060079 Sources: GOC:BHF Also known as: negative regulation of excitatory post-synaptic membrane potential, reduction of excitatory postsynaptic membrane potential, negative regulation of EPSP